N-cyclopropylmelamine deaminase activity [GO:0034547] (molecular function) Sources: UM-BBD_reactionID:r0825 Definition: Catalysis of the reaction: cyromazine + H2O = N-cyclopropylammeline + NH3. Relationships: is_a hydrolase activity, acting on carbon-nitrogen (but not peptide) bonds, in cyclic amidines [GO:0016814]